arsenate reductase activity [GO:0030611] (molecular function) Definition: Catalysis of the reaction: arsenite + A + H2O = arsenate + AH2 + H+. Also known as: arsenate reductase (donor) activity, arsenate:(acceptor) oxidoreductase activity, arsenate:acceptor oxidoreductase activity Sources: RHEA:18449 Relationships: is a type of oxidoreductase activity, acting on phosphorus or arsenic in donors [GO:0030613]